{
  "term_id": "GO:0006955",
  "gene": "UniProtKB:P30511",
  "gene_name": "HLA class I histocompatibility antigen, alpha chain F",
  "gene_symbol": "HLA-F",
  "term_label": "immune response"
}